negative regulation of myeloid cell apoptotic process [GO:0033033] (biological process) Subtypes: negative regulation of mast cell apoptotic process [GO:0033026], negative regulation of neutrophil apoptotic process [GO:0033030], negative regulation of erythrocyte apoptotic process [GO:1902251], GO:2000110 Also known as: down regulation of myeloid cell apoptosis, down-regulation of myeloid cell apoptosis, downregulation of myeloid cell apoptosis, inhibition of myeloid cell apoptosis, negative regulation of myeloid cell apoptosis Definition: Any process that stops, prevents, or reduces the frequency, rate, or extent of a myeloid cell apoptotic process. Sources: GOC:add, GOC:mtg_apoptosis Relationships: is a type of regulation of myeloid cell apoptotic process [GO:0033032]; is a type of negative regulation of apoptotic process [GO:0043066]; negatively regulates GO:0033028